{
  "gene_name": "Olfactory receptor 4F4",
  "gene": "UniProtKB:Q96R69",
  "term_label": "Unknown biological process",
  "term_id": "UNKNOWN:0002",
  "gene_symbol": "OR4F4"
}